{
  "gene_name": "Beta-hexosaminidase subunit beta",
  "term_id": "GO:0030203",
  "gene": "UniProtKB:P07686",
  "term_label": "glycosaminoglycan metabolic process",
  "gene_symbol": "HEXB"
}